retrograde transport, vacuole to Golgi [GO:0045018] (biological process) Also known as: retrograde transport from the vacuole Relationships: is a type of vacuolar transport [GO:0007034] References: PMID:9700156 Definition: The directed movement of substances from the vacuole to the trans-Golgi network; this occurs in yeast via the prevacuolar/endosomal compartment.